{
  "gene_name": "Cadherin-4",
  "gene_symbol": "CDH4",
  "term_label": "cell-cell junction assembly",
  "gene": "UniProtKB:P55283",
  "term_id": "GO:0007043"
}